tyramine secretion [GO:0061545] (biological process) Definition: The regulated release of a tyramine by a cell. Sources: GOC:dph Relationships: is a type of monoamine transport [GO:0015844]; is a type of organic hydroxy compound transport [GO:0015850]; is a type of primary amine secretion [GO:0061531] Subtypes: GO:0061546